alanine-glyoxylate transaminase activity [GO:0008453] (molecular function) Also known as: alanine-glyoxylate aminotransferase activity, AGT activity, L-alanine-glycine transaminase activity, L-alanine:glyoxylate aminotransferase activity, alanine--glyoxylate aminotransferase activity, alanine-glyoxylic aminotransferase activity Definition: Catalysis of the reaction: L-alanine + glyoxylate = pyruvate + glycine. Relationships: is a type of transaminase activity [GO:0008483] Sources: EC:2.6.1.44